mesenchymal cell migration [GO:0090497] (biological process) Definition: The orderly movement of a mesenchymal cell from one site to another, often during the development of a multicellular organism. Relationships: is a type of GO:0001667 Sources: GOC:dph, GOC:tb Subtypes: neural crest cell migration [GO:0001755], GO:0035322